sperm mitochondrial sheath [GO:0097226] (cellular component) Definition: The tightly packed helical sheath of ATP-producing mitochondria restricted to the midpiece of the sperm flagellum. References: PMID:32791035 Sources: GOC:cjm, MP:0009832 Relationships: is a type of cellular anatomical structure [GO:0110165]; is part of sperm midpiece [GO:0097225]